sensory neuron migration [GO:1904937] (biological process) Relationships: is a type of neuron migration [GO:0001764] References: PMID:18622031 Sources: GOC:TermGenie, GOC:ah, GO_REF:0000091 Definition: The orderly movement of a sensory neuron from one site to another.